MIM complex [GO:0140595] (CC) Sources: GOC:vw Also known as: mitochondrial outer import machinery Relationships: is a type of outer mitochondrial membrane protein complex [GO:0098799] Definition: A protein complex located in the mitochondrial outer membrane that functions as an insertase, mediating the insertion of alpha-helical proteins from the cytosol into the outer membrane. Client proteins are usually single- and multi-span proteins that include components of the TOM complex.